{
  "term_label": "plasma membrane",
  "gene": "UniProtKB:Q9UM73",
  "gene_symbol": "ALK",
  "gene_name": "ALK tyrosine kinase receptor",
  "term_id": "GO:0005886"
}